{
  "gene": "UniProtKB:O15427",
  "gene_symbol": "SLC16A3",
  "term_id": "GO:0016323",
  "gene_name": "Monocarboxylate transporter 4",
  "term_label": "basolateral plasma membrane"
}